glycerol-3-phosphate-transporting ATPase complex [GO:1902517] (cellular component) Note: An example of this is UgpB in E. coli in PMID:23013274. Relationships: is a type of ATP-binding cassette (ABC) transporter complex [GO:0043190] Definition: A protein complex which is capable of glycerol-3-phosphate-transporting ATPase activity. References: PMID:23013274 Sources: GOC:TermGenie, GOC:bhm